positive regulation of pigment cell differentiation [GO:0050942] (BP) Definition: Any process that activates or increases the frequency, rate or extent of pigment cell differentiation. Sources: GOC:ai Also known as: up regulation of pigment cell differentiation, up-regulation of pigment cell differentiation, upregulation of pigment cell differentiation, activation of pigment cell differentiation, stimulation of pigment cell differentiation Relationships: is a type of GO:0045597; is_a positive regulation of developmental pigmentation [GO:0048087]; is a type of regulation of pigment cell differentiation [GO:0050932]; positively regulates GO:0050931 Subtypes: GO:0045636, GO:0048777, positive regulation of erythrophore differentiation [GO:0048780], positive regulation of cyanophore differentiation [GO:0048783], positive regulation of iridophore differentiation [GO:0050945], positive regulation of xanthophore differentiation [GO:0050946]